maintenance of DNA trinucleotide repeats [GO:0035753] (biological process) Relationships: is a type of maintenance of DNA repeat elements [GO:0043570] References: PMID:21347277 Sources: GOC:rb, SO:0000291 Definition: Any process involved in sustaining the fidelity and copy number of DNA trinucleotide repeats. DNA trinucleotide repeats are naturally occurring runs of three base-pairs.